{
  "term_id": "GO:0097242",
  "gene": "UniProtKB:P21757",
  "term_label": "amyloid-beta clearance",
  "gene_symbol": "MSR1",
  "gene_name": "Macrophage scavenger receptor types I and II"
}